{
  "gene_symbol": "PPARG",
  "term_id": "GO:0006631",
  "gene": "UniProtKB:P37231",
  "term_label": "fatty acid metabolic process",
  "gene_name": "Peroxisome proliferator-activated receptor gamma"
}